cellular response to fatty acid [GO:0071398] (biological process) Relationships: is a type of GO:0070542; is a type of GO:0071396; is a type of cellular response to oxygen-containing compound [GO:1901701] Definition: Any process that results in a change in state or activity of a cell (in terms of movement, secretion, enzyme production, gene expression, etc.) as a result of a fatty acid stimulus. Sources: GOC:mah Subtypes: cellular response to jasmonic acid stimulus [GO:0071395], GO:0071399, cellular response to oleic acid [GO:0071400], cellular response to leptomycin B [GO:0072750], cellular response to lipoic acid [GO:1903443], GO:1903545, cellular response to arachidonate [GO:1904551], cellular response to ionomycin [GO:1904637], cellular response to palmitoleic acid [GO:1904927], GO:1905390